{
  "gene": "UniProtKB:Q9BVQ7",
  "term_label": "autophagosome maturation",
  "gene_symbol": "AFG2B",
  "term_id": "GO:0097352",
  "gene_name": "ATPase family gene 2 protein homolog B"
}